adhesion of symbiont to microvasculature [GO:0020035] (biological process) References: PMID:10362584 Sources: GOC:mb Relationships: is a type of adhesion of symbiont to host cell [GO:0044650] Also known as: symbiont-protein-mediated cytoadherence to microvasculature, cytoadherence to microvasculature, mediated by symbiont protein, cytoadherence to microvasculature, mediated by parasite protein, heterophilic cell adhesion involved in cytoadherence to microvasculature, mediated by parasite protein, parasite-protein-mediated cytoadherence to microvasculature Definition: The adherence of symbiont-infected erythrocytes to microvascular endothelium via symbiont proteins embedded in the membrane of the erythrocyte.